{
  "gene_symbol": "PYGB",
  "term_label": "pyridoxal phosphate binding",
  "gene": "UniProtKB:P11216",
  "term_id": "GO:0030170",
  "gene_name": "Glycogen phosphorylase, brain form"
}